regulation of photorespiration [GO:0080093] (biological process) Sources: GOC:tb Relationships: is a type of regulation of biosynthetic process [GO:0009889]; RO_0002211 photorespiration [GO:0009853] Definition: Any process that modulates the rate, frequency or extent of photorespiration. Photorespiration is a light-dependent catabolic process occurring concomitantly with photosynthesis in plants (especially C3 plants) whereby dioxygen (O2) is consumed and carbon dioxide (CO2) is evolved.